negative regulation of placenta blood vessel development [GO:0110081] (biological process) Definition: Any process that stops, prevents or reduces the frequency, rate or extent of placenta blood vessel development. References: PMID:27748453 Sources: GOC:BHF, GOC:BHF_miRNA, GOC:rph Relationships: is a type of negative regulation of developmental process [GO:0051093]; is_a regulation of placenta blood vessel development [GO:0110079]; negatively regulates placenta blood vessel development [GO:0060674]